{
  "gene_symbol": "FXYD5",
  "gene_name": "FXYD domain-containing ion transport regulator 5",
  "term_label": "sodium channel regulator activity",
  "term_id": "GO:0017080",
  "gene": "UniProtKB:Q96DB9"
}